{
  "gene_name": "Alpha-N-acetylgalactosaminide alpha-2,6-sialyltransferase 3",
  "gene_symbol": "ST6GALNAC3",
  "term_id": "GO:0001574",
  "term_label": "ganglioside biosynthetic process",
  "gene": "UniProtKB:Q8NDV1"
}